lysosome to ER cholesterol transport [GO:0090120] (biological process) Relationships: is a type of lysosomal transport [GO:0007041]; is a type of GO:0016192; is a type of intracellular cholesterol transport [GO:0032367]; occurs in cytoplasm [GO:0005737] Also known as: lysosome to endoplasmic reticulum cholesterol transport Sources: GOC:mah Definition: The directed movement of cholesterol, cholest-5-en-3-beta-ol, or cholesterol-containing compounds, from the lysosome to the endoplasmic reticulum.